{
  "term_label": "plasma membrane",
  "term_id": "GO:0005886",
  "gene_symbol": "OR5V1",
  "gene": "UniProtKB:Q9UGF6",
  "gene_name": "Olfactory receptor 5V1"
}